{
  "gene_symbol": "ATPSCKMT",
  "gene_name": "ATP synthase subunit C lysine N-methyltransferase",
  "term_id": "GO:1905706",
  "term_label": "regulation of mitochondrial ATP synthesis coupled proton transport",
  "gene": "UniProtKB:Q6P4H8"
}